isopropylmalate transport [GO:0034659] (biological process) Sources: GOC:mah Subtypes: GO:1902357 Relationships: is_a dicarboxylic acid transport [GO:0006835]; is a type of GO:0015718; is a type of GO:0015850 Definition: The directed movement of isopropylmalate into, out of or within a cell, or between cells, by means of some agent such as a transporter or pore.